{
  "term_label": "Unknown cellular component",
  "gene_symbol": "MKRN3",
  "term_id": "UNKNOWN:0003",
  "gene": "UniProtKB:Q13064",
  "gene_name": "Probable E3 ubiquitin-protein ligase makorin-3"
}